{
  "gene": "UniProtKB:O75554",
  "term_label": "RNA splicing",
  "term_id": "GO:0008380",
  "gene_symbol": "WBP4",
  "gene_name": "WW domain-binding protein 4"
}